regulation of cytokine activity [GO:0060300] (biological process) Subtypes: negative regulation of cytokine activity [GO:0060302], regulation of chemokine activity [GO:1900136] Sources: GOC:BHF, GOC:dph, GOC:tb Relationships: is a type of GO:0010469; is a type of regulation of receptor binding [GO:1900120]; regulates GO:0005125 Definition: Any process that modulates the rate, frequency or extent of the activity of a molecule that controls the survival, growth, differentiation and effector function of tissues and cells.